regulation of male gonad development [GO:2000018] (biological process) Definition: Any process that modulates the frequency, rate or extent of male gonad development. Sources: GOC:obol, GOC:yaf Also known as: regulation of testicular development, regulation of testis development Relationships: is a type of GO:1905939; regulates male gonad development [GO:0008584] Subtypes: negative regulation of male gonad development [GO:2000019], positive regulation of male gonad development [GO:2000020]